positive regulation of adipose tissue development [GO:1904179] (biological process) References: PMID:23081848 Sources: GOC:TermGenie, GO_REF:0000058 Relationships: is a type of positive regulation of developmental process [GO:0051094]; is a type of positive regulation of multicellular organismal process [GO:0051240]; is_a regulation of adipose tissue development [GO:1904177]; positively regulates adipose tissue development [GO:0060612] Definition: Any process that activates or increases the frequency, rate or extent of adipose tissue development. Also known as: up regulation of adipose tissue development, up-regulation of adipose tissue development, upregulation of adipose tissue development, activation of adipose tissue development, activation of adipogenesis, positive regulation of adipogenesis, up regulation of adipogenesis, up-regulation of adipogenesis, upregulation of adipogenesis